response to growth hormone [GO:0060416] (biological process) Definition: Any process that results in a change in state or activity of a cell or an organism (in terms of movement, secretion, enzyme production, gene expression, etc.) as a result of a growth hormone stimulus. Growth hormone is a peptide hormone that binds to the growth hormone receptor and stimulates growth. Sources: GOC:BHF, GOC:dph Also known as: response to growth hormone stimulus Relationships: is a type of response to peptide hormone [GO:0043434] Subtypes: cellular response to growth hormone stimulus [GO:0071378]